{
  "gene_symbol": "WNT3",
  "term_id": "GO:0045165",
  "gene": "UniProtKB:P56703",
  "term_label": "cell fate commitment",
  "gene_name": "Proto-oncogene Wnt-3"
}